RNA guanosine-uridine insertion [GO:0070714] (biological process) Definition: The modification of an RNA molecule by insertion of an guanosine-uridine insertion dinucleotide. Also known as: RNA GU insertion Relationships: is a type of RNA dinucleotide insertion [GO:0070707] Sources: GOC:cb, GOC:mah